{
  "term_id": "GO:0005737",
  "term_label": "cytoplasm",
  "gene": "UniProtKB:Q8NI29",
  "gene_name": "F-box only protein 27",
  "gene_symbol": "FBXO27"
}